positive regulation of secretory granule organization [GO:1904411] (biological process) Definition: Any process that activates or increases the frequency, rate or extent of secretory granule organization. Also known as: positive regulation of secretory granule organisation, up regulation of secretory granule organisation, up regulation of secretory granule organization, up-regulation of secretory granule organisation, up-regulation of secretory granule organization, upregulation of secretory granule organisation, upregulation of secretory granule organization, activation of secretory granule organisation, activation of secretory granule organization, activation of secretory granule organization and biogenesis, positive regulation of secretory granule organization and biogenesis, up regulation of secretory granule organization and biogenesis, up-regulation of secretory granule organization and biogenesis, upregulation of secretory granule organization and biogenesis Relationships: is a type of positive regulation of organelle organization [GO:0010638]; is a type of regulation of secretory granule organization [GO:1904409]; positively regulates secretory granule organization [GO:0033363] References: PMID:15039777 Sources: GOC:TermGenie, GO_REF:0000058